negative regulation of entry of bacterium into host cell [GO:2000536] (biological process) Relationships: is a type of negative regulation of biological process [GO:0048519]; is a type of GO:2000535; negatively regulates GO:0035635 Also known as: negative regulation of bacterial entry into host cell, negative regulation of invasion of bacteria into host cell Sources: GOC:obol Definition: Any process that stops, prevents or reduces the frequency, rate or extent of entry of bacterium into host cell.